allantoin transport [GO:0015720] (BP) Definition: The directed movement of allantoin, (2,5-dioxo-4-imidazolidinyl)urea, into, out of or within a cell, or between cells, by means of some agent such as a transporter or pore. Relationships: is a type of amide transport [GO:0042886] Also known as: allantoin/allantoate transport, allantoin transmembrane transport Sources: GOC:ai